{
  "term_id": "GO:0043066",
  "gene_name": "Baculoviral IAP repeat-containing protein 5",
  "term_label": "negative regulation of apoptotic process",
  "gene": "UniProtKB:O15392",
  "gene_symbol": "BIRC5"
}